{
  "gene_symbol": "DNAI2",
  "term_label": "dynein light chain binding",
  "gene_name": "Dynein axonemal intermediate chain 2",
  "gene": "UniProtKB:Q9GZS0",
  "term_id": "GO:0045503"
}